{
  "gene_name": "Death domain-associated protein 6",
  "term_label": "nuclear androgen receptor binding",
  "term_id": "GO:0050681",
  "gene_symbol": "DAXX",
  "gene": "UniProtKB:Q9UER7"
}